regulation of neutrophil mediated killing of symbiont cell [GO:0070949] (biological process) Sources: GOC:add, GOC:mah Definition: Any process that modulates the rate, frequency or extent of neutrophil mediated killing of a symbiont cell, the directed killing of a symbiont target cell by a neutrophil. Relationships: is a type of regulation of response to biotic stimulus [GO:0002831]; is a type of regulation of defense response [GO:0031347]; is a type of regulation of response to external stimulus [GO:0032101]; is a type of GO:0043903; is a type of GO:0051709; is_a regulation of neutrophil mediated cytotoxicity [GO:0070948]; regulates neutrophil-mediated killing of symbiont cell [GO:0070943] Subtypes: regulation of neutrophil mediated killing of bacterium [GO:0070950], GO:0070953, negative regulation of neutrophil mediated killing of symbiont cell [GO:0070955], GO:0070961